{
  "gene_symbol": "ALKBH7",
  "gene_name": "Alpha-ketoglutarate-dependent dioxygenase alkB homolog 7, mitochondrial",
  "term_label": "fatty acid metabolic process",
  "term_id": "GO:0006631",
  "gene": "UniProtKB:Q9BT30"
}